{
  "term_id": "GO:0008541",
  "gene": "UniProtKB:O43242",
  "gene_symbol": "PSMD3",
  "gene_name": "26S proteasome non-ATPase regulatory subunit 3",
  "term_label": "proteasome regulatory particle, lid subcomplex"
}